regulation of cytoplasmic mRNA processing body assembly [GO:0010603] (biological process) Relationships: is a type of regulation of organelle assembly [GO:1902115]; regulates P-body assembly [GO:0033962] Definition: Any process that modulates the rate, frequency, or extent of the aggregation, arrangement and bonding together of proteins and RNA molecules to form a cytoplasmic mRNA processing body. Subtypes: GO:0010606, GO:0010607 Sources: GOC:dph, GOC:krc, GOC:tb